{
  "term_label": "AP-type membrane coat adaptor complex",
  "term_id": "GO:0030119",
  "gene_symbol": "AP5M1",
  "gene": "UniProtKB:Q9H0R1",
  "gene_name": "AP-5 complex subunit mu-1"
}